{
  "term_label": "endoplasmic reticulum membrane",
  "gene_symbol": "RTN1",
  "term_id": "GO:0005789",
  "gene": "UniProtKB:Q16799",
  "gene_name": "Reticulon-1"
}